{
  "gene_name": "F-box only protein 27",
  "gene_symbol": "FBXO27",
  "term_label": "ERAD pathway",
  "gene": "UniProtKB:Q8NI29",
  "term_id": "GO:0036503"
}